{
  "term_label": "negative regulation of epidermal growth factor receptor signaling pathway",
  "term_id": "GO:0042059",
  "gene_name": "Protein sprouty homolog 1",
  "gene_symbol": "SPRY1",
  "gene": "UniProtKB:O43609"
}